{
  "term_label": "Unknown molecular function",
  "term_id": "UNKNOWN:0001",
  "gene": "UniProtKB:Q15008",
  "gene_name": "26S proteasome non-ATPase regulatory subunit 6",
  "gene_symbol": "PSMD6"
}